kidney mesenchymal cell proliferation [GO:0072135] (biological process) Subtypes: mesonephric mesenchymal cell proliferation involved in mesonephros development [GO:0061222], metanephric mesenchymal cell proliferation involved in metanephros development [GO:0072136] Definition: The multiplication or reproduction of cells, resulting in the expansion of a mesenchymal cell population in the kidney. Relationships: is a type of mesenchymal cell proliferation [GO:0010463]; is a type of cell proliferation involved in kidney development [GO:0072111]; is part of kidney mesenchyme development [GO:0072074] Sources: GOC:mtg_kidney_jan10